{
  "gene_name": "Heart- and neural crest derivatives-expressed protein 2",
  "term_id": "GO:0007507",
  "term_label": "heart development",
  "gene": "UniProtKB:P61296",
  "gene_symbol": "HAND2"
}